{
  "term_label": "nucleus",
  "term_id": "GO:0005634",
  "gene": "UniProtKB:Q12774",
  "gene_name": "Rho guanine nucleotide exchange factor 5",
  "gene_symbol": "ARHGEF5"
}